conversion of glutamyl-tRNA to glutaminyl-tRNA [GO:0043685] (biological process) References: PMID:3340166, PMID:9342308 Sources: GOC:jsg Definition: The modification process that results in the conversion of glutamate charged on a tRNA(Gln) to glutaminyl-tRNA. Relationships: is a type of charged-tRNA amino acid modification [GO:0019988] Note: Note that this process has been observed in some archaeal and bacterial species.